sterigmatocystin 7-O-methyltransferase activity [GO:0047146] (molecular function) Sources: EC:2.1.1.110, MetaCyc:2.1.1.110-RXN Also known as: O-methyltransferase II activity, S-adenosyl-L-methionine:sterigmatocystin 7-O-methyltransferase activity, S-adenosyl-L-methionine:sterigmatocystin 8-O-methyltransferase activity, sterigmatocystin 8-O-methyltransferase activity, sterigmatocystin methyltransferase activity Definition: Catalysis of the reaction: sterigmatocystin + S-adenosyl-L-methionine = 7-O-methylsterigmatocystin + S-adenosyl-homocysteine. Relationships: is a type of O-methyltransferase activity [GO:0008171]